Bam protein complex [GO:1990063] (cellular component) References: PMID:20378773 Sources: GOC:bhm Relationships: is a type of membrane protein complex [GO:0098796]; is part of GO:0031241 Definition: Protein complex which is involved in assembly and insertion of beta-barrel proteins into the outer membrane. In E. coli it is composed of BamABCDE, of the outer membrane protein BamA, and four lipoproteins BamB, BamC, BamD and BamE. BamA interacts directly with BamB and the BamCDE subcomplex. Also known as: OMP complex